negative regulation of nonadec-1-ene biosynthetic process [GO:1900936] (biological process) Also known as: down regulation of nonadec-1-ene anabolism, down regulation of nonadec-1-ene biosynthesis, down regulation of nonadec-1-ene biosynthetic process, down regulation of nonadec-1-ene formation, down regulation of nonadec-1-ene synthesis, down-regulation of nonadec-1-ene anabolism, down-regulation of nonadec-1-ene biosynthesis, down-regulation of nonadec-1-ene biosynthetic process, down-regulation of nonadec-1-ene formation, down-regulation of nonadec-1-ene synthesis, downregulation of nonadec-1-ene anabolism, downregulation of nonadec-1-ene biosynthesis, downregulation of nonadec-1-ene biosynthetic process, downregulation of nonadec-1-ene formation, downregulation of nonadec-1-ene synthesis, inhibition of nonadec-1-ene anabolism, inhibition of nonadec-1-ene biosynthesis, inhibition of nonadec-1-ene formation, inhibition of nonadec-1-ene synthesis, negative regulation of nonadec-1-ene anabolism, negative regulation of nonadec-1-ene biosynthesis, negative regulation of nonadec-1-ene formation, negative regulation of nonadec-1-ene synthesis, inhibition of nonadec-1-ene biosynthetic process Relationships: is a type of negative regulation of olefin biosynthetic process [GO:1900912]; is_a regulation of nonadec-1-ene biosynthetic process [GO:1900935]; negatively regulates nonadec-1-ene biosynthetic process [GO:1900877] Definition: Any process that stops, prevents or reduces the frequency, rate or extent of nonadec-1-ene biosynthetic process. Sources: GOC:TermGenie, GOC:mengo_curators